archaeal or bacterial-type flagellum-dependent cell motility [GO:0097588] (biological process) Definition: Cell motility due to movement of bacterial- or archaeal-type flagella. Relationships: is a type of GO:0001539 Subtypes: bacterial-type flagellum-dependent cell motility [GO:0071973], archaeal-type flagellum-dependent cell motility [GO:0097590] Note: Bacterial- and archaeal-type flagella are superficially similar but have a different molecular composition and fine structure. This term was added for mapping to the UniProt keyword "flagellar rotation". For manual annotation, please use one of the child terms of GO:0097588 that refer specifically to either archaeal- or bacterial-type flagella. Sources: GOC:cilia, GOC:krc